chitin biosynthetic process [GO:0006031] (biological process) Relationships: is a type of aminoglycan biosynthetic process [GO:0006023]; is a type of chitin metabolic process [GO:0006030]; is a type of glucosamine-containing compound biosynthetic process [GO:1901073] Also known as: beta-1,4-linked N-acetylglucosamine biosynthesis, beta-1,4-linked N-acetylglucosamine biosynthetic process, chitin anabolism, chitin biosynthesis, chitin formation, chitin synthesis Sources: GOC:jl, ISBN:0198506732 Definition: The chemical reactions and pathways resulting in the formation of chitin, a linear polysaccharide consisting of beta-(1->4)-linked N-acetyl-D-glucosamine residues. Regulation: regulated by regulation of chitin biosynthetic process [GO:0032883]